beta-tubulin binding [GO:0048487] (molecular function) Also known as: beta tubulin binding Definition: Binding to the microtubule constituent protein beta-tubulin. Relationships: is a type of tubulin binding [GO:0015631] Sources: GOC:krc